forebrain induction by the anterior neural ridge [GO:0022000] (biological process) Relationships: is a type of developmental induction [GO:0031128]; is part of neural plate anterior/posterior regionalization [GO:0021999] Sources: GOC:cls, GOC:dgh, GOC:dph, GOC:jid, GO_REF:0000021 Definition: The close range interaction of the anterior neural ridge to the caudal region of the neural plate that specifies the forebrain fate.